{
  "gene_name": "Ras-related protein Rab-4A",
  "term_label": "insulin-responsive compartment",
  "gene": "UniProtKB:P20338",
  "term_id": "GO:0032593",
  "gene_symbol": "RAB4A"
}